ganglion mother cell fate determination [GO:0007402] (biological process) Definition: The cell fate determination process in which a cell becomes capable of differentiating autonomously into a ganglion mother cell regardless of its environment; upon determination, the cell fate cannot be reversed. Sources: GOC:go_curators Relationships: is a type of GO:0001709